{
  "term_id": "GO:0005783",
  "term_label": "endoplasmic reticulum",
  "gene_symbol": "ZDHHC22",
  "gene_name": "Palmitoyltransferase ZDHHC22",
  "gene": "UniProtKB:Q8N966"
}